cristae formation [GO:0042407] (biological process) Sources: GOC:jl, ISBN:0198506732 Definition: The assembly of cristae, the inwards folds of the inner mitochondrial membrane. Regulation: regulated by regulation of cristae formation [GO:1903850]; negatively regulated by negative regulation of cristae formation [GO:1903851]; positively regulated by positive regulation of cristae formation [GO:1903852] Relationships: is_a inner mitochondrial membrane organization [GO:0007007]